{
  "term_id": "GO:0043161",
  "term_label": "proteasome-mediated ubiquitin-dependent protein catabolic process",
  "gene": "UniProtKB:Q5VWM6",
  "gene_symbol": "PRAMEF13",
  "gene_name": "Putative PRAME family member 13"
}